L-serine ammonia-lyase activity [GO:0003941] (molecular function) Sources: EC:4.3.1.17 Also known as: L-hydroxyaminoacid dehydratase activity, L-serine dehydratase activity, serine deaminase activity, L-serine deaminase activity, L-serine hydro-lyase (deaminating) activity, L-serine ammonia-lyase (pyruvate-forming) activity, L-serine dehydration activity Relationships: is a type of ammonia-lyase activity [GO:0016841] Definition: Catalysis of the reaction: L-serine = pyruvate + NH3.